{
  "gene": "UniProtKB:P55036",
  "gene_name": "26S proteasome non-ATPase regulatory subunit 4",
  "gene_symbol": "PSMD4",
  "term_id": "GO:0043161",
  "term_label": "proteasome-mediated ubiquitin-dependent protein catabolic process"
}